{
  "gene_symbol": "PDCD7",
  "term_id": "UNKNOWN:0002",
  "gene_name": "Programmed cell death protein 7",
  "gene": "UniProtKB:Q8N8D1",
  "term_label": "Unknown biological process"
}